glutamine secretion [GO:0010585] (biological process) Relationships: is a type of glutamine transport [GO:0006868]; is a type of secretion by cell [GO:0032940] References: PMID:15208395 Definition: The controlled release of glutamine by a cell.